sclerenchyma cell differentiation [GO:0014001] (biological process) Relationships: is a type of cell differentiation [GO:0030154] Regulation: regulated by regulation of sclerenchyma cell differentiation [GO:1904368]; positively regulated by positive regulation of sclerenchyma cell differentiation [GO:1904369] Definition: The process in which a relatively unspecialized cell acquires specialized features of a sclerenchyma cell. A sclerenchyma cell is a plant cell with thick lignified walls, normally dead at maturity and specialized for structural strength. Includes fiber cells, that are greatly elongated; and sclereids, that are more isodiametric. Intermediate types exist. Cells may or may not be devoid of protoplasm at maturity. Cell form and size are variable. Sources: CL:0000276, GOC:ef, GOC:jid, PO:0000077